ribonucleoprotein complex [GO:1990904] (cellular component) Also known as: RNA-protein complex, RNP, protein-RNA complex, extracellular ribonucleoprotein complex, intracellular ribonucleoprotein complex Definition: A macromolecular complex that contains both RNA and protein molecules. Relationships: is a type of protein-containing complex [GO:0032991] Subtypes: GO:0005681, telomerase holoenzyme complex [GO:0005697], GO:0005732, X chromosome located dosage compensation complex, transcription activating [GO:0016456], small nuclear ribonucleoprotein complex [GO:0030532], ribonuclease P complex [GO:0030677], preribosome [GO:0030684], GO:0031332, Mei2 nuclear dot complex [GO:0033620], multi-eIF complex [GO:0043614], translation initiation ternary complex [GO:0044207], ribosomal subunit [GO:0044391], signal recognition particle [GO:0048500], Smp focus [GO:0062238], pre-snoRNP complex [GO:0070761], GO:0070992, cytosolic translation preinitiation complex [GO:0070993], histone pre-mRNA 3'end processing complex [GO:0071204], mitochondrial translation preinitiation complex [GO:0180053], GO:1990572 Sources: GOC:krc, GOC:vesicles